{
  "gene_name": "Dual specificity protein kinase TTK",
  "term_label": "protein localization to kinetochore",
  "gene": "UniProtKB:P33981",
  "gene_symbol": "TTK",
  "term_id": "GO:0034501"
}